neurotransmitter receptor transport, plasma membrane to endosome [GO:0099646] (biological process) Sources: GOC:dos Definition: Vesicle-mediated transport of a neurotransmitter receptor vesicle from the plasma membrane to the endosome. Relationships: is a type of protein localization to endosome [GO:0036010]; is a type of GO:0048227; is a type of establishment of protein localization to organelle [GO:0072594]; is a type of GO:0099637